arrestin family protein binding [GO:1990763] (molecular function) Relationships: is a type of protein binding [GO:0005515] References: PMID:23911909 Definition: Binding to a member of the arrestin family, proteins involved in agonist-mediated desensitization of G protein-coupled receptors.